anaerobic gallate catabolic process [GO:0019328] (biological process) Also known as: anaerobic gallate breakdown, anaerobic gallate catabolism, anaerobic gallate degradation, anaerobic gallic acid catabolic process, anaerobic gallic acid catabolism, gallate fermentation Sources: GOC:jl Relationships: is a type of gallate catabolic process [GO:0019396] Definition: The chemical reactions and pathways resulting in the breakdown of gallate, the anion of gallic acid, in the absence of oxygen.